{
  "gene_name": "Inorganic pyrophosphatase",
  "gene": "UniProtKB:Q15181",
  "gene_symbol": "PPA1",
  "term_id": "GO:0004427",
  "term_label": "inorganic diphosphate phosphatase activity"
}